pyridoxamine-phosphate transaminase activity [GO:0019163] (molecular function) Definition: Catalysis of the reaction: pyridoxamine 5'-phosphate + 2-oxoglutarate = pyridoxal 5'-phosphate + D-glutamate. Also known as: pyridoxamine-phosphate aminotransferase activity, pyridoxamine 5'-phosphate transaminase activity, pyridoxamine 5'-phosphate-alpha-ketoglutarate transaminase activity, pyridoxamine phosphate aminotransferase activity, pyridoxamine-5'-phosphate:2-oxoglutarate aminotransferase (D-glutamate-forming) Sources: EC:2.6.1.54 Relationships: is_a GO:0008483